myotube cell migration [GO:0110122] (biological process) Definition: The orderly movement of a myotube cell from one site to another, often during the development of a multicellular organism. Myotubes are multinucleated cells that are formed when proliferating myoblasts exit the cell cycle, differentiate, and fuse. Relationships: is a type of muscle cell migration [GO:0014812] Regulation: regulated by GO:0110123; positively regulated by GO:0110124; negatively regulated by negative regulation of myotube cell migration [GO:0110125] References: PMID:29122742 Sources: GOC:ha Subtypes: GO:1904969